integrin alpha7-beta1 complex [GO:0034677] (cellular component) Relationships: is_a integrin complex [GO:0008305] References: PMID:12297042 Also known as: alpha7-beta1 integrin complex, ITGA7-ITGB1 complex Definition: An integrin complex that comprises one alpha7 subunit and one beta1 subunit.